adenylate cyclase-activating adrenergic receptor signaling pathway involved in heart process [GO:0086023] (biological process) Also known as: adrenergic receptor signaling pathway involved in heart process, adrenergic receptor signalling pathway involved in heart process, beta-adrenergic receptor signalling pathway involved in heart process Sources: GOC:BHF, GOC:mtg_cardiac_conduct_nov11 Relationships: is a type of GO:0071880; is a type of GO:0086103 Subtypes: adenylate cyclase-activating adrenergic receptor signaling pathway involved in cardiac muscle relaxation [GO:0086030] Regulation: positively regulated by positive regulation of adenylate cyclase-activating adrenergic receptor signaling pathway involved in heart process [GO:0140196]; negatively regulated by negative regulation of adenylate cyclase-activating adrenergic receptor signaling pathway involved in heart process [GO:0140199] Definition: The series of molecular signals beginning with a G protein-coupled adrenergic cell surface receptor combining with epinephrine or norepinephrine, to activate adenylate cyclase, which contributes to a circulatory system process carried out by the heart.